{
  "gene": "UniProtKB:P45452",
  "term_id": "GO:0005615",
  "gene_name": "Collagenase 3",
  "gene_symbol": "MMP13",
  "term_label": "extracellular space"
}